{
  "gene": "UniProtKB:Q9UHF3",
  "gene_name": "Putative N-acetyltransferase 8B",
  "term_label": "N-acetyltransferase activity",
  "gene_symbol": "NAT8B",
  "term_id": "GO:0008080"
}